{
  "gene": "UniProtKB:A6NJI9",
  "term_label": "Unknown molecular function",
  "gene_symbol": "LRRC72",
  "gene_name": "Leucine-rich repeat-containing protein 72",
  "term_id": "UNKNOWN:0001"
}